{
  "term_id": "UNKNOWN:0001",
  "gene": "UniProtKB:C9JVW0",
  "gene_name": "Putative transmembrane protein INAFM1",
  "gene_symbol": "INAFM1",
  "term_label": "Unknown molecular function"
}